regulation of budding cell apical bud growth [GO:0010568] (biological process) Definition: Any process that modulates the frequency, rate or extent of growth at the tip of a bud, in a cell that reproduces by budding. Relationships: is_a regulation of growth [GO:0040008]; regulates budding cell apical bud growth [GO:0007118] References: PMID:17417630 Sources: GOC:dph, GOC:jp, GOC:tb